{
  "term_id": "GO:0030881",
  "gene_name": "HLA class I histocompatibility antigen, B alpha chain",
  "gene_symbol": "HLA-B",
  "term_label": "beta-2-microglobulin binding",
  "gene": "UniProtKB:P01889"
}